{
  "gene_name": "Rhomboid-related protein 1",
  "gene_symbol": "RHBDL1",
  "term_id": "UNKNOWN:0003",
  "gene": "UniProtKB:O75783",
  "term_label": "Unknown cellular component"
}